protein-glutamic acid ligase activity, initiating [GO:0106437] (molecular function) References: PMID:32747782 Sources: RHEA:60144 Relationships: is a type of GO:0070739 Definition: Catalytic reaction: ATP + L-glutamate + L-glutamyl-[protein] = ADP + H+ + L-gamma-glutamyl-L-glutamyl-[protein] + phosphate.